{
  "gene": "UniProtKB:Q99962",
  "term_label": "protein-macromolecule adaptor activity",
  "term_id": "GO:0030674",
  "gene_name": "Endophilin-A1",
  "gene_symbol": "SH3GL2"
}